{
  "term_id": "GO:0016485",
  "term_label": "protein processing",
  "gene_symbol": "TMPRSS11E",
  "gene_name": "Transmembrane protease serine 11E",
  "gene": "UniProtKB:Q9UL52"
}